uronolactonase activity [GO:0050389] (molecular function) Also known as: D-glucurono-6,2-lactone lactonohydrolase activity, glucuronolactonase activity Relationships: is a type of carboxylic ester hydrolase activity [GO:0052689] Sources: EC:3.1.1.19, MetaCyc:URONOLACTONASE-RXN Definition: Catalysis of the reaction: D-glucurono-6,2-lactone + H2O = D-glucuronate.